{
  "term_id": "GO:1904263",
  "gene": "UniProtKB:Q8N3F9",
  "term_label": "positive regulation of TORC1 signaling",
  "gene_symbol": "GPR137C",
  "gene_name": "Integral membrane protein GPR137C"
}